{
  "term_label": "Unknown molecular function",
  "gene_symbol": "CATSPERZ",
  "term_id": "UNKNOWN:0001",
  "gene_name": "Cation channel sperm-associated auxiliary subunit zeta",
  "gene": "UniProtKB:Q9NTU4"
}